{
  "term_id": "GO:0007608",
  "term_label": "sensory perception of smell",
  "gene": "UniProtKB:Q8NGG6",
  "gene_name": "Olfactory receptor 8B12",
  "gene_symbol": "OR8B12"
}